{
  "gene_name": "Heparan sulfate glucosamine 3-O-sulfotransferase 4",
  "gene": "UniProtKB:Q9Y661",
  "gene_symbol": "HS3ST4",
  "term_id": "GO:0008467",
  "term_label": "[heparan sulfate]-glucosamine 3-sulfotransferase activity"
}